{
  "gene": "UniProtKB:Q5JST6",
  "term_label": "regulation of dendrite morphogenesis",
  "gene_symbol": "EFHC2",
  "term_id": "GO:0048814",
  "gene_name": "EF-hand domain-containing family member C2"
}